{
  "gene_name": "Heat shock factor protein 5",
  "term_id": "GO:0003700",
  "gene_symbol": "HSF5",
  "gene": "UniProtKB:Q4G112",
  "term_label": "DNA-binding transcription factor activity"
}